{
  "term_id": "GO:0005874",
  "gene_symbol": "KIF16B",
  "term_label": "microtubule",
  "gene_name": "Kinesin-like protein KIF16B",
  "gene": "UniProtKB:Q96L93"
}